aflatoxin metabolic process [GO:0046222] (biological process) Subtypes: aflatoxin biosynthetic process [GO:0045122], aflatoxin catabolic process [GO:0046223] Definition: The chemical reactions and pathways involving aflatoxin, a fungal metabolite found as a contaminant in moldy grains that induces liver cancer. Aflatoxin induces a G to T transversion at codon 249 of p53, leading to its inactivation. Aflatoxin is converted to a chemical carcinogen by P450. Sources: GOC:ai Also known as: aflatoxin metabolism, aflatoxin B metabolic process, aflatoxin B1 metabolic process, aflatoxin B1 metabolism, aflatoxin B2 metabolic process, aflatoxin B2 metabolism Relationships: is a type of mycotoxin metabolic process [GO:0043385]